{
  "term_id": "UNKNOWN:0003",
  "gene_name": "Immunoglobulin V-set domain-containing protein (Fragment)",
  "term_label": "Unknown cellular component",
  "gene": "UniProtKB:A0A0J9YW62",
  "gene_symbol": "A0A0J9YW62"
}